{
  "gene": "UniProtKB:Q32MQ0",
  "term_label": "RNA polymerase II cis-regulatory region sequence-specific DNA binding",
  "term_id": "GO:0000978",
  "gene_symbol": "ZNF750",
  "gene_name": "Zinc finger protein 750"
}